{
  "term_label": "plasma membrane",
  "gene": "UniProtKB:Q9P0J7",
  "gene_name": "E3 ubiquitin-protein ligase KCMF1",
  "gene_symbol": "KCMF1",
  "term_id": "GO:0005886"
}